positive regulation of ecdysteroid secretion [GO:0046000] (biological process) Relationships: is a type of regulation of ecdysteroid secretion [GO:0007555]; is a type of positive regulation of steroid hormone secretion [GO:2000833]; positively regulates ecdysteroid secretion [GO:0045457] Definition: Any process that activates or increases the frequency, rate or extent of the regulated release of ecdysteroid. Also known as: up regulation of ecdysteroid secretion, up-regulation of ecdysteroid secretion, upregulation of ecdysteroid secretion, activation of ecdysteroid secretion, stimulation of ecdysteroid secretion Sources: GOC:go_curators